{
  "gene": "UniProtKB:Q8NGT5",
  "term_id": "UNKNOWN:0001",
  "gene_name": "Olfactory receptor 9A2",
  "gene_symbol": "OR9A2",
  "term_label": "Unknown molecular function"
}